{
  "gene_symbol": "TNF",
  "term_id": "GO:2001238",
  "term_label": "positive regulation of extrinsic apoptotic signaling pathway",
  "gene": "UniProtKB:P01375",
  "gene_name": "Tumor necrosis factor"
}